{
  "gene": "UniProtKB:Q9H2V7",
  "gene_symbol": "SPNS1",
  "gene_name": "Protein spinster homolog 1",
  "term_id": "GO:0051977",
  "term_label": "lysophospholipid transport"
}